mitotic nuclear bridge [GO:0140510] (cellular component) Relationships: is a type of cellular anatomical structure [GO:0110165]; BFO_0000050 nucleus [GO:0005634] References: PMID:32848252 Also known as: nuclear bridge Definition: A narrow constricted region of the nucleus that forms around the anaphase spindle during closed mitosis, and connects the main portions of the newly forming daughter nuclei.